{
  "gene": "UniProtKB:P78332",
  "term_id": "GO:0003723",
  "gene_name": "RNA-binding protein 6",
  "gene_symbol": "RBM6",
  "term_label": "RNA binding"
}